transcription pausing by RNA polymerase II [GO:0160239] (biological process) Definition: A transcription halt following transcription initiation but prior to elongation, during which RNA polymerase II pauses approximately 20-60 nucleotides downstream of the transcriptional start site before proceeding into productive elongation. Transcription pausing starts following phosphorylation of the C-terminal domain (CTD) of RNA polymerase II subunit POLR2A at Ser-5 and stops following phosphorylation of POLR2A by the P-TEFb complex. Relationships: is a type of RNA biosynthetic process [GO:0032774]; is part of transcription by RNA polymerase II [GO:0006366] Also known as: promoter proximal pausing by RNA polymerase II References: PMID:33271312, PMID:35816930